{
  "gene_symbol": "UGT1A8",
  "gene_name": "UDP-glucuronosyltransferase 1A8",
  "term_label": "endoplasmic reticulum",
  "gene": "UniProtKB:Q9HAW9",
  "term_id": "GO:0005783"
}